cellobiose transport [GO:0019533] (biological process) Definition: The directed movement of cellobiose into, out of or within a cell, or between cells, by means of some agent such as a transporter or pore. Cellobiose, or 4-O-beta-D-glucopyranosyl-D-glucose, is a disaccharide that represents the basic repeating unit of cellulose. Sources: GOC:ai Relationships: is a type of disaccharide transport [GO:0015766]